linoleic acid epoxygenase activity [GO:0071614] (molecular function) Relationships: is a type of monooxygenase activity [GO:0004497]; is a type of oxidoreductase activity, acting on paired donors, with incorporation or reduction of molecular oxygen [GO:0016705] Definition: Catalysis of an NADPH- and oxygen-dependent reaction that converts linoleic acid to a cis-epoxyoctadecenoic acid. Also known as: linoleic acid monooxygenase activity References: PMID:11042099 Sources: GOC:BHF